{
  "term_id": "GO:0035372",
  "gene_symbol": "MID2",
  "gene": "UniProtKB:Q9UJV3",
  "term_label": "protein localization to microtubule",
  "gene_name": "Probable E3 ubiquitin-protein ligase MID2"
}